{
  "gene": "UniProtKB:Q96AJ9",
  "term_id": "GO:0016236",
  "gene_name": "Vesicle transport through interaction with t-SNAREs homolog 1A",
  "term_label": "macroautophagy",
  "gene_symbol": "VTI1A"
}